{
  "gene_name": "Zinc finger protein Helios",
  "gene_symbol": "IKZF2",
  "term_id": "GO:0003700",
  "term_label": "DNA-binding transcription factor activity",
  "gene": "UniProtKB:Q9UKS7"
}